{
  "term_id": "UNKNOWN:0003",
  "gene_symbol": "OTUB1",
  "term_label": "Unknown cellular component",
  "gene_name": "Ubiquitin thioesterase OTUB1",
  "gene": "UniProtKB:Q96FW1"
}